carboxy-terminal domain protein kinase complex [GO:0032806] (cellular component) Definition: A protein complex that phosphorylates amino acid residues of RNA polymerase II C-terminal domain repeats; phosphorylation occurs mainly on Ser2 and Ser5. References: PMID:15047695, PMID:16721054, PMID:17079683 Also known as: CTDK complex Relationships: is_a nuclear protein-containing complex [GO:0140513]; is a type of serine/threonine protein kinase complex [GO:1902554] Subtypes: transcription factor TFIIH holo complex [GO:0005675], cyclin/CDK positive transcription elongation factor complex [GO:0008024]